{
  "gene_name": "Testis anion transporter 1",
  "gene_symbol": "SLC26A8",
  "term_label": "sulfate transmembrane transporter activity",
  "term_id": "GO:0015116",
  "gene": "UniProtKB:Q96RN1"
}